{
  "gene_name": "NKG2-D type II integral membrane protein",
  "term_id": "GO:0038023",
  "gene_symbol": "KLRK1",
  "gene": "UniProtKB:P26718",
  "term_label": "signaling receptor activity"
}